{
  "term_label": "protein localization to nuclear inner membrane",
  "term_id": "GO:0036228",
  "gene_symbol": "NUP54",
  "gene_name": "Nucleoporin p54",
  "gene": "UniProtKB:Q7Z3B4"
}